regulation of hydrolase activity [GO:0051336] (biological process) Also known as: hydrolase regulator Sources: GOC:ai Definition: Any process that modulates the frequency, rate or extent of hydrolase activity, the catalysis of the hydrolysis of various bonds, e.g. C-O, C-N, C-C, phosphoric anhydride bonds, etc. Hydrolase is the systematic name for any enzyme of EC class 3. Relationships: is a type of regulation of catalytic activity [GO:0050790]; regulates hydrolase activity [GO:0016787] Subtypes: regulation of phospholipase activity [GO:0010517], regulation of phosphatase activity [GO:0010921], regulation of beta-lactamase activity [GO:0033252], GO:0043087, positive regulation of hydrolase activity [GO:0051345], negative regulation of hydrolase activity [GO:0051346], regulation of peptidase activity [GO:0052547]